actin cytoskeleton of dendritic spine [GO:0098938] (cellular component) Relationships: is a type of cytoskeleton of dendritic spine [GO:0098836]; is a type of GO:0098871 Sources: GOC:dos Definition: The actin cytoskeleton that is part of a dendritic spine.